{
  "gene": "UniProtKB:Q8NGY3",
  "term_id": "GO:0004984",
  "gene_name": "Olfactory receptor 6K3",
  "term_label": "olfactory receptor activity",
  "gene_symbol": "OR6K3"
}